{
  "term_id": "GO:0005634",
  "gene_symbol": "USP11",
  "gene": "UniProtKB:P51784",
  "gene_name": "Ubiquitin carboxyl-terminal hydrolase 11",
  "term_label": "nucleus"
}